{
  "term_label": "nucleus",
  "gene_symbol": "UBE2L5",
  "gene": "UniProtKB:A0A1B0GUS4",
  "gene_name": "Ubiquitin-conjugating enzyme E2 L5",
  "term_id": "GO:0005634"
}